{
  "gene": "UniProtKB:Q9NTJ5",
  "gene_name": "Phosphatidylinositol-3-phosphatase SAC1",
  "term_label": "endoplasmic reticulum",
  "gene_symbol": "SACM1L",
  "term_id": "GO:0005783"
}